{
  "gene_name": "Nicotinamide_nicotinic acid mononucleotide adenylyltransferase 3",
  "gene": "UniProtKB:Q96T66",
  "gene_symbol": "NMNAT3",
  "term_id": "GO:0034355",
  "term_label": "NAD+ biosynthetic process via the salvage pathway"
}